{
  "gene_name": "Uncharacterized protein C2orf80",
  "term_id": "UNKNOWN:0002",
  "gene_symbol": "C2orf80",
  "gene": "UniProtKB:Q0P641",
  "term_label": "Unknown biological process"
}